{
  "term_id": "GO:0006888",
  "gene": "UniProtKB:Q9Y3Q3",
  "gene_symbol": "TMED3",
  "gene_name": "Transmembrane emp24 domain-containing protein 3",
  "term_label": "endoplasmic reticulum to Golgi vesicle-mediated transport"
}